{
  "gene_name": "LIM domain-binding protein 2",
  "gene": "UniProtKB:O43679",
  "gene_symbol": "LDB2",
  "term_id": "GO:0005634",
  "term_label": "nucleus"
}